regulation of small intestinal transit [GO:0120057] (BP) Subtypes: positive regulation of small intestinal transit [GO:0120058], negative regulation of small intestinal transit [GO:0120059] References: PMID:15890336 Sources: GOC:sl Relationships: is a type of regulation of digestive system process [GO:0044058]; regulates small intestinal transit [GO:0120055] Also known as: regulation of small bowel transit, regulation of small intestine transit Definition: Any process that modulates the frequency, rate or extent of any small intestinal transit process, the migration of ingested material along the length of the small intestine.